{
  "gene_symbol": "DDAH2",
  "gene_name": "N(G),N(G)-dimethylarginine dimethylaminohydrolase 2",
  "gene": "UniProtKB:O95865",
  "term_id": "UNKNOWN:0001",
  "term_label": "Unknown molecular function"
}